{
  "gene": "UniProtKB:Q7Z443",
  "gene_name": "Polycystin-1-like protein 3",
  "term_label": "detection of mechanical stimulus",
  "term_id": "GO:0050982",
  "gene_symbol": "PKD1L3"
}